{
  "gene_symbol": "DST",
  "term_id": "GO:0005882",
  "gene_name": "Dystonin",
  "term_label": "intermediate filament",
  "gene": "UniProtKB:Q03001"
}